{
  "term_id": "GO:0048015",
  "gene": "UniProtKB:P48736",
  "term_label": "phosphatidylinositol-mediated signaling",
  "gene_symbol": "PIK3CG",
  "gene_name": "Phosphatidylinositol 4,5-bisphosphate 3-kinase catalytic subunit gamma isoform"
}